{
  "gene_symbol": "AJM1",
  "gene": "UniProtKB:C9J069",
  "gene_name": "Apical junction component 1 homolog",
  "term_label": "Unknown molecular function",
  "term_id": "UNKNOWN:0001"
}